{
  "gene_name": "Contactin-6",
  "term_id": "GO:0070593",
  "gene": "UniProtKB:Q9UQ52",
  "term_label": "dendrite self-avoidance",
  "gene_symbol": "CNTN6"
}